{
  "gene_symbol": "LCN9",
  "gene": "UniProtKB:Q8WX39",
  "term_id": "UNKNOWN:0002",
  "gene_name": "Epididymal-specific lipocalin-9",
  "term_label": "Unknown biological process"
}